{
  "gene": "UniProtKB:Q9HAA7",
  "gene_symbol": "Q9HAA7",
  "term_label": "Unknown biological process",
  "gene_name": "Putative uncharacterized protein FLJ11871",
  "term_id": "UNKNOWN:0002"
}